purine ribonucleoside diphosphate metabolic process [GO:0009179] (biological process) Subtypes: purine ribonucleoside diphosphate biosynthetic process [GO:0009180], purine ribonucleoside diphosphate catabolic process [GO:0009181], GO:0046031, IDP metabolic process [GO:0046707], GDP metabolic process [GO:0046710] Also known as: purine ribonucleoside diphosphate metabolism Definition: The chemical reactions and pathways involving purine ribonucleoside diphosphate, a compound consisting of a purine base linked to a ribose sugar esterified with diphosphate on the sugar. Relationships: is_a purine nucleoside diphosphate metabolic process [GO:0009135]; is a type of GO:0009185 Sources: GOC:go_curators, ISBN:0198506732